{
  "gene_symbol": "AKNAD1",
  "term_label": "Unknown molecular function",
  "gene": "UniProtKB:Q5T1N1",
  "term_id": "UNKNOWN:0001",
  "gene_name": "Protein AKNAD1"
}